poly(U) RNA binding [GO:0008266] (molecular function) Sources: GOC:mah Relationships: is a type of GO:0008187 Also known as: poly(U) binding Definition: Binding to a sequence of uracil residues in an RNA molecule.